{
  "gene": "UniProtKB:P57077",
  "gene_name": "MAP3K7 C-terminal-like protein",
  "term_label": "Unknown cellular component",
  "term_id": "UNKNOWN:0003",
  "gene_symbol": "MAP3K7CL"
}